fluoride export across plasma membrane [GO:0140116] (biological process) Relationships: is a type of GO:0140115; is a type of fluoride transmembrane transport [GO:1903424] Definition: The directed movement of fluoride ions from inside of a cell, across the plasma membrane and into the extracellular region. References: PMID:27327046 Sources: GOC:vw